RNA polymerase III transcription repressor complex [GO:0090572] (cellular component) Relationships: is a type of GO:0017053; is a type of nuclear protein-containing complex [GO:0140513] Sources: GOC:tb Definition: A protein complex, located in the nucleus, that possesses activity that prevents or downregulates transcription from a RNA polymerase III promoter.